{
  "term_label": "DNA-binding transcription factor activity, RNA polymerase II-specific",
  "term_id": "GO:0000981",
  "gene": "UniProtKB:Q9C0A1",
  "gene_symbol": "ZFHX2",
  "gene_name": "Zinc finger homeobox protein 2"
}